gastrin-releasing peptide receptor binding [GO:0031709] (molecular function) Sources: GOC:mah, GOC:nln Definition: Binding to a gastrin-releasing peptide receptor. Relationships: is a type of bombesin receptor binding [GO:0031705] Also known as: GRP receptor binding, gastrin-releasing peptide receptor ligand